{
  "gene": "UniProtKB:P42262",
  "term_label": "dendritic spine",
  "gene_symbol": "GRIA2",
  "gene_name": "Glutamate receptor 2",
  "term_id": "GO:0043197"
}